regulation of mRNA export from nucleus [GO:0010793] (biological process) Subtypes: GO:2000728 Definition: Any process that modulates the frequency, rate or extent of the directed movement of mRNA from the nucleus to the cytoplasm. Relationships: is a type of regulation of RNA export from nucleus [GO:0046831]; is a type of regulation of ribonucleoprotein complex localization [GO:2000197]; regulates mRNA export from nucleus [GO:0006406] Sources: GOC:dph, GOC:tb